{
  "gene_symbol": "TAF5",
  "term_id": "GO:0005669",
  "gene_name": "Transcription initiation factor TFIID subunit 5",
  "term_label": "transcription factor TFIID complex",
  "gene": "UniProtKB:Q15542"
}